{
  "gene_symbol": "MAMDC2",
  "gene_name": "MAM domain-containing protein 2",
  "term_label": "Unknown cellular component",
  "gene": "UniProtKB:Q7Z304",
  "term_id": "UNKNOWN:0003"
}